{
  "term_label": "Unknown cellular component",
  "gene_name": "Zinc finger protein 667",
  "term_id": "UNKNOWN:0003",
  "gene_symbol": "ZNF667",
  "gene": "UniProtKB:Q5HYK9"
}